{
  "gene": "UniProtKB:Q13496",
  "term_label": "phosphatidylinositol dephosphorylation",
  "term_id": "GO:0046856",
  "gene_symbol": "MTM1",
  "gene_name": "Myotubularin"
}